{
  "term_label": "B cell activation involved in immune response",
  "gene_name": "Interferon alpha-1_13",
  "term_id": "GO:0002312",
  "gene": "UniProtKB:P01562",
  "gene_symbol": "IFNA1"
}